equator specification [GO:0045317] (biological process) Relationships: is a type of formation of anatomical boundary [GO:0048859]; BFO_0000050 GO:0042067 Definition: The formation and development of the equator that forms the boundary between the photoreceptors in the dorsal sector of the eye and those in the ventral sector, dividing the eye into dorsal and ventral halves. Sources: GOC:bf